{
  "term_id": "GO:0005943",
  "term_label": "phosphatidylinositol 3-kinase complex, class IA",
  "gene_symbol": "PIK3CA",
  "gene": "UniProtKB:P42336",
  "gene_name": "Phosphatidylinositol 4,5-bisphosphate 3-kinase catalytic subunit alpha isoform"
}